negative regulation of transcription regulatory region DNA binding [GO:2000678] (biological process) Sources: GOC:obol Relationships: is a type of negative regulation of DNA binding [GO:0043392]; is a type of regulation of transcription regulatory region DNA binding [GO:2000677]; negatively regulates transcription cis-regulatory region binding [GO:0000976] Definition: Any process that stops, prevents or reduces the frequency, rate or extent of transcription regulatory region DNA binding. Subtypes: negative regulation of RNA polymerase II regulatory region sequence-specific DNA binding [GO:1903026], negative regulation of core promoter binding [GO:1904797]